{
  "gene": "UniProtKB:O75899",
  "term_id": "GO:0038039",
  "gene_symbol": "GABBR2",
  "term_label": "G protein-coupled receptor heterodimeric complex",
  "gene_name": "Gamma-aminobutyric acid type B receptor subunit 2"
}